peptidyl-methionine modification [GO:0018206] (biological process) Sources: GOC:go_curators Definition: The modification of peptidyl-methionine. Subtypes: N-terminal peptidyl-methionine acetylation [GO:0017196] Relationships: is a type of peptidyl-amino acid modification [GO:0018193]